{
  "term_label": "plasma membrane",
  "gene": "UniProtKB:Q9Y5I1",
  "gene_name": "Protocadherin alpha-11",
  "gene_symbol": "PCDHA11",
  "term_id": "GO:0005886"
}